{
  "gene": "UniProtKB:Q9UI12",
  "term_id": "UNKNOWN:0001",
  "term_label": "Unknown molecular function",
  "gene_name": "V-type proton ATPase subunit H",
  "gene_symbol": "ATP6V1H"
}